{
  "gene_symbol": "CTSF",
  "term_id": "GO:0005764",
  "gene_name": "Cathepsin F",
  "gene": "UniProtKB:Q9UBX1",
  "term_label": "lysosome"
}